{
  "gene": "UniProtKB:Q86WV6",
  "term_id": "GO:0045087",
  "gene_name": "Stimulator of interferon genes protein",
  "gene_symbol": "STING1",
  "term_label": "innate immune response"
}